{
  "gene_symbol": "TRAM2",
  "gene_name": "Translocating chain-associated membrane protein 2",
  "term_label": "Unknown molecular function",
  "term_id": "UNKNOWN:0001",
  "gene": "UniProtKB:Q15035"
}